histone H3K9cr reader activity [GO:0140019] (MF) Also known as: H3K9cr modified histone binding References: PMID:27105114 Definition: A histone reader that recognizes a histone H3 crotonylated at lysine 9. Relationships: is_a GO:0140006 Note: Comment: Note that the residue position corresponds to the canonical human H3 histone (UniProtKB:P84243); this residue is conserved across all eukaryotes. Residue 1 is the first residue following removal of the initiating Methionine (Met). Note that each histone is encoded by multiple genes, and sequences may vary across different genes within an organism.